{
  "gene_symbol": "FGB",
  "term_label": "blood coagulation, fibrin clot formation",
  "gene": "UniProtKB:P02675",
  "gene_name": "Fibrinogen beta chain",
  "term_id": "GO:0072378"
}